{
  "gene": "UniProtKB:Q96N21",
  "term_id": "UNKNOWN:0002",
  "gene_name": "AP-4 complex accessory subunit Tepsin",
  "term_label": "Unknown biological process",
  "gene_symbol": "TEPSIN"
}